mitotic DNA damage checkpoint signaling [GO:0044773] (biological process) Sources: GOC:TermGenie, GOC:mtg_cell_cycle Also known as: intracellular signaling cascade involved in mitotic DNA damage checkpoint, mitotic DNA damage checkpoint, signal transduction involved in mitotic DNA damage checkpoint, intracellular signal transduction pathway involved in mitotic DNA damage checkpoint, intracellular signaling pathway involved in mitotic DNA damage checkpoint Definition: A signal transduction process involved in mitotic DNA damage checkpoint. Subtypes: mitotic G2 DNA damage checkpoint signaling [GO:0007095], mitotic G1 DNA damage checkpoint signaling [GO:0031571], mitotic intra-S DNA damage checkpoint signaling [GO:0031573] Relationships: is a type of DNA damage checkpoint signaling [GO:0000077]; is a type of mitotic DNA integrity checkpoint signaling [GO:0044774] Regulation: regulated by regulation of mitotic DNA damage checkpoint [GO:1904289]; negatively regulated by negative regulation of mitotic DNA damage checkpoint [GO:1904290]; positively regulated by GO:1904291